{
  "gene_name": "Small integral membrane protein 40",
  "term_id": "UNKNOWN:0003",
  "term_label": "Unknown cellular component",
  "gene": "UniProtKB:Q5STR5",
  "gene_symbol": "SMIM40"
}